{
  "gene_name": "Tumor necrosis factor receptor superfamily member 10B",
  "term_label": "positive regulation of apoptotic process",
  "gene": "UniProtKB:O14763",
  "gene_symbol": "TNFRSF10B",
  "term_id": "GO:0043065"
}